{
  "term_id": "GO:0007060",
  "gene_symbol": "TEX11",
  "gene_name": "Testis-expressed protein 11",
  "term_label": "male meiosis chromosome segregation",
  "gene": "UniProtKB:Q8IYF3"
}